{
  "term_label": "synaptic transmission, glutamatergic",
  "gene": "UniProtKB:Q9UPW8",
  "gene_symbol": "UNC13A",
  "term_id": "GO:0035249",
  "gene_name": "Protein unc-13 homolog A"
}